{
  "gene_name": "SHC-transforming protein 4",
  "term_label": "cell surface receptor protein tyrosine kinase signaling pathway",
  "term_id": "GO:0007169",
  "gene_symbol": "SHC4",
  "gene": "UniProtKB:Q6S5L8"
}